{
  "gene_name": "Mothers against decapentaplegic homolog 7",
  "gene_symbol": "SMAD7",
  "term_id": "GO:0140416",
  "gene": "UniProtKB:O15105",
  "term_label": "transcription regulator inhibitor activity"
}